{
  "gene": "UniProtKB:P05108",
  "gene_symbol": "CYP11A1",
  "term_label": "glucocorticoid biosynthetic process",
  "term_id": "GO:0006704",
  "gene_name": "Cholesterol side-chain cleavage enzyme, mitochondrial"
}